negative regulation of innate immunity memory response [GO:1905681] (biological process) Definition: Any process that stops, prevents or reduces the frequency, rate or extent of innate immunity memory response. Sources: GOC:TermGenie, GO_REF:0000058 Also known as: down regulation of innate immunity memory response, down-regulation of innate immunity memory response, downregulation of innate immunity memory response, inhibition of innate immunity memory response Relationships: is a type of GO:0045824; is a type of GO:1905680; negatively regulates innate immunity memory response [GO:0090714]